{
  "gene_name": "Na(+)_citrate cotransporter",
  "term_id": "GO:0015746",
  "gene_symbol": "SLC13A5",
  "gene": "UniProtKB:Q86YT5",
  "term_label": "citrate transport"
}